negative regulation of mitotic centrosome separation [GO:0046603] (BP) Relationships: is a type of negative regulation of cell cycle process [GO:0010948]; is a type of GO:0046602; negatively regulates mitotic centrosome separation [GO:0007100] Sources: GOC:ai Also known as: down regulation of mitotic centrosome separation, down-regulation of mitotic centrosome separation, downregulation of mitotic centrosome separation, inhibition of mitotic centrosome separation Definition: Any process that stops, prevents, or reduces the frequency, rate or extent of centrosome separation.